{
  "term_label": "Unknown molecular function",
  "gene": "UniProtKB:Q9Y291",
  "gene_name": "Small ribosomal subunit protein mS33",
  "gene_symbol": "MRPS33",
  "term_id": "UNKNOWN:0001"
}